positive regulation of emericellamide A biosynthetic process [GO:1900663] (biological process) Also known as: activation of emericellamide A anabolism, activation of emericellamide A biosynthesis, activation of emericellamide A formation, activation of emericellamide A synthesis, positive regulation of emericellamide A anabolism, positive regulation of emericellamide A biosynthesis, positive regulation of emericellamide A formation, positive regulation of emericellamide A synthesis, up regulation of emericellamide A anabolism, up regulation of emericellamide A biosynthesis, up regulation of emericellamide A biosynthetic process, up regulation of emericellamide A formation, up regulation of emericellamide A synthesis, up-regulation of emericellamide A anabolism, up-regulation of emericellamide A biosynthesis, up-regulation of emericellamide A biosynthetic process, up-regulation of emericellamide A formation, up-regulation of emericellamide A synthesis, upregulation of emericellamide A anabolism, upregulation of emericellamide A biosynthesis, upregulation of emericellamide A biosynthetic process, upregulation of emericellamide A formation, upregulation of emericellamide A synthesis, activation of emericellamide A biosynthetic process Definition: Any process that activates or increases the frequency, rate or extent of emericellamide A biosynthetic process. Sources: GOC:TermGenie, GOC:di Relationships: is a type of GO:1900660; is a type of regulation of emericellamide A biosynthetic process [GO:1900661]; positively regulates emericellamide A biosynthetic process [GO:1900617]